{
  "gene_name": "Intraflagellar transport protein 88 homolog",
  "term_label": "kinesin binding",
  "gene": "UniProtKB:Q13099",
  "term_id": "GO:0019894",
  "gene_symbol": "IFT88"
}